{
  "gene_name": "Major histocompatibility complex class I-related gene protein",
  "gene": "UniProtKB:Q95460",
  "gene_symbol": "MR1",
  "term_id": "GO:0005615",
  "term_label": "extracellular space"
}